{
  "term_id": "GO:0050839",
  "gene_symbol": "PCDHGA2",
  "gene_name": "Protocadherin gamma-A2",
  "term_label": "cell adhesion molecule binding",
  "gene": "UniProtKB:Q9Y5H1"
}